{
  "term_id": "GO:0032020",
  "term_label": "ISG15-protein conjugation",
  "gene_symbol": "UBE2E2",
  "gene_name": "Ubiquitin-conjugating enzyme E2 E2",
  "gene": "UniProtKB:Q96LR5"
}